{
  "term_id": "GO:0016303",
  "gene_symbol": "PIK3C3",
  "term_label": "1-phosphatidylinositol-3-kinase activity",
  "gene_name": "Phosphatidylinositol 3-kinase catalytic subunit type 3",
  "gene": "UniProtKB:Q8NEB9"
}